{
  "gene": "UniProtKB:Q86YF9",
  "term_label": "ciliary basal body",
  "gene_symbol": "DZIP1",
  "gene_name": "Cilium assembly protein DZIP1",
  "term_id": "GO:0036064"
}